{
  "gene": "UniProtKB:Q9BUT1",
  "gene_symbol": "BDH2",
  "gene_name": "Dehydrogenase_reductase SDR family member 6",
  "term_id": "GO:0005737",
  "term_label": "cytoplasm"
}